{
  "gene_symbol": "IGHV3-64",
  "gene": "UniProtKB:A0A075B6Q5",
  "gene_name": "Immunoglobulin heavy variable 3-64",
  "term_id": "GO:0003823",
  "term_label": "antigen binding"
}